{
  "term_label": "RNA endonuclease activity",
  "gene_name": "Uridylate-specific endoribonuclease",
  "term_id": "GO:0004521",
  "gene": "UniProtKB:P21128",
  "gene_symbol": "ENDOU"
}